negative regulation of cardiac muscle cell proliferation [GO:0060044] (biological process) Definition: Any process that stops, prevents, or reduces the frequency, rate or extent of cardiac muscle cell proliferation. Sources: GOC:dph, GOC:rph Also known as: negative regulation of heart muscle cell proliferation Relationships: is a type of negative regulation of cell population proliferation [GO:0008285]; is a type of negative regulation of cardiac muscle tissue growth [GO:0055022]; is a type of regulation of cardiac muscle cell proliferation [GO:0060043]; negatively regulates cardiac muscle cell proliferation [GO:0060038]